{
  "term_id": "GO:0005634",
  "gene_symbol": "SPATA33",
  "term_label": "nucleus",
  "gene": "UniProtKB:Q96N06",
  "gene_name": "Spermatogenesis-associated protein 33"
}